{
  "term_label": "glucosyltransferase activity",
  "gene_name": "Protein O-glucosyltransferase 3",
  "gene_symbol": "POGLUT3",
  "gene": "UniProtKB:Q7Z4H8",
  "term_id": "GO:0046527"
}